{
  "gene": "UniProtKB:Q86TJ5",
  "gene_name": "Zinc finger protein 554",
  "term_label": "regulation of transcription by RNA polymerase II",
  "term_id": "GO:0006357",
  "gene_symbol": "ZNF554"
}